{
  "gene": "UniProtKB:Q16570",
  "term_id": "UNKNOWN:0003",
  "term_label": "Unknown cellular component",
  "gene_name": "Atypical chemokine receptor 1",
  "gene_symbol": "ACKR1"
}